{
  "term_id": "GO:0038111",
  "gene_name": "Interleukin-7 receptor subunit alpha",
  "gene": "UniProtKB:P16871",
  "term_label": "interleukin-7-mediated signaling pathway",
  "gene_symbol": "IL7R"
}